{
  "gene_name": "DNA excision repair protein ERCC-1",
  "term_id": "GO:0006312",
  "gene_symbol": "ERCC1",
  "gene": "UniProtKB:P07992",
  "term_label": "mitotic recombination"
}